{
  "term_label": "detection of chemical stimulus involved in sensory perception of smell",
  "gene_name": "Olfactory receptor 2T3",
  "term_id": "GO:0050911",
  "gene": "UniProtKB:Q8NH03",
  "gene_symbol": "OR2T3"
}